{
  "term_id": "GO:0005737",
  "gene_symbol": "GHDC",
  "gene_name": "GH3 domain-containing protein",
  "gene": "UniProtKB:Q8N2G8",
  "term_label": "cytoplasm"
}